{
  "gene": "UniProtKB:Q9UH65",
  "gene_symbol": "SWAP70",
  "term_id": "GO:0005737",
  "term_label": "cytoplasm",
  "gene_name": "Switch-associated protein 70"
}